negative regulation of protein export from nucleus [GO:0046826] (biological process) Also known as: down regulation of protein export from nucleus, down-regulation of protein export from nucleus, downregulation of protein export from nucleus, negative regulation of protein export from cell nucleus, negative regulation of protein export out of nucleus, negative regulation of protein transport from nucleus to cytoplasm, negative regulation of protein-nucleus export, inhibition of protein export from nucleus Relationships: is a type of GO:0046823; is a type of regulation of protein export from nucleus [GO:0046825]; is a type of GO:0051457; is_a negative regulation of intracellular protein transport [GO:0090317]; negatively regulates protein export from nucleus [GO:0006611] Definition: Any process that stops, prevents, or reduces the frequency, rate or extent of the directed movement of proteins from the nucleus into the cytoplasm. Sources: GOC:bf